CD154 receptor binding [GO:0042615] (molecular function) Definition: Binding to CD154, a receptor found on the surface of some activated lymphocytes. Sources: GOC:jl, ISBN:0120781859 Also known as: CD40L binding, CD40 receptor activity Relationships: is a type of signaling receptor binding [GO:0005102]